{
  "gene_name": "Apoptosis-inducing factor 1, mitochondrial",
  "gene": "UniProtKB:O95831",
  "gene_symbol": "AIFM1",
  "term_id": "GO:0005739",
  "term_label": "mitochondrion"
}